gentisate decarboxylase activity [GO:0047923] (molecular function) Sources: EC:4.1.1.62, RHEA:21312 Definition: Catalysis of the reaction: 2,5-dihydroxybenzoate + H+ = CO2 + hydroquinone. Also known as: 2,5-dihydroxybenzoate carboxy-lyase (hydroquinone-forming), 2,5-dihydroxybenzoate decarboxylase activity, gentisate carboxy-lyase activity Relationships: is a type of carboxy-lyase activity [GO:0016831]